{
  "term_label": "L-ascorbate:sodium symporter activity",
  "gene": "UniProtKB:Q9UGH3",
  "gene_name": "Solute carrier family 23 member 2",
  "term_id": "GO:0008520",
  "gene_symbol": "SLC23A2"
}